{
  "gene_name": "Probable glucose sensor protein SLC5A4",
  "term_id": "GO:0035623",
  "gene_symbol": "SLC5A4",
  "gene": "UniProtKB:Q9NY91",
  "term_label": "renal D-glucose absorption"
}